{
  "gene_name": "Sperm-associated antigen 1",
  "term_label": "Unknown molecular function",
  "gene_symbol": "SPAG1",
  "term_id": "UNKNOWN:0001",
  "gene": "UniProtKB:Q07617"
}